peptide-N4-(N-acetyl-beta-glucosaminyl)asparagine amidase activity [GO:0000224] (molecular function) Definition: Catalysis of the reaction: 4-N-(N-acetyl-D-glucosaminyl)-protein + H2O = N-acetyl-beta-D-glucosaminylamine + peptide L-aspartate. This reaction is the hydrolysis of an N4-(acetyl-beta-D-glucosaminyl)asparagine residue in which the N-acetyl-D-glucosamine residue may be further glycosylated, to yield a (substituted) N-acetyl-beta-D-glucosaminylamine and the peptide containing an aspartic residue. Also known as: glycopeptidase activity, glycopeptide N-glycosidase activity, PNGase, jack-bean glycopeptidase, N-glycanase activity, N-linked-glycopeptide-(N-acetyl-beta-D-glucosaminyl)-L-asparagine amidohydrolase activity, N-oligosaccharide glycopeptidase activity, PNGase A, PNGase F, peptide:N-glycanase Relationships: is a type of hydrolase activity, acting on carbon-nitrogen (but not peptide) bonds, in linear amides [GO:0016811] Sources: EC:3.5.1.52